negative regulation of antimicrobial peptide biosynthetic process [GO:0002806] (biological process) Relationships: is a type of negative regulation of antimicrobial peptide production [GO:0002785]; is a type of regulation of antimicrobial peptide biosynthetic process [GO:0002805]; negatively regulates antimicrobial peptide biosynthetic process [GO:0002777] Subtypes: negative regulation of antibacterial peptide biosynthetic process [GO:0002809], negative regulation of antifungal peptide biosynthetic process [GO:0002811] Also known as: down regulation of antimicrobial peptide biosynthetic process, down-regulation of antimicrobial peptide biosynthetic process, downregulation of antimicrobial peptide biosynthetic process, inhibition of antimicrobial peptide biosynthetic process Definition: Any process that stops, prevents, or reduces the frequency, rate, or extent of antimicrobial peptide biosynthesis. Sources: GOC:add